{
  "gene_name": "Interleukin-24",
  "term_label": "immune response",
  "gene": "UniProtKB:Q13007",
  "term_id": "GO:0006955",
  "gene_symbol": "IL24"
}